{
  "gene_symbol": "DAPP1",
  "gene_name": "Dual adapter for phosphotyrosine and 3-phosphotyrosine and 3-phosphoinositide",
  "term_label": "phospholipid binding",
  "gene": "UniProtKB:Q9UN19",
  "term_id": "GO:0005543"
}